negative regulation of T cell proliferation [GO:0042130] (biological process) Also known as: down regulation of T cell proliferation, down-regulation of T cell proliferation, downregulation of T cell proliferation, negative regulation of T lymphocyte proliferation, negative regulation of T-cell proliferation, negative regulation of T-lymphocyte proliferation, inhibition of T cell proliferation Sources: GOC:jl Definition: Any process that stops, prevents or reduces the rate or extent of T cell proliferation. Relationships: is a type of GO:0042129; is a type of negative regulation of lymphocyte proliferation [GO:0050672]; is a type of negative regulation of T cell activation [GO:0050868]; negatively regulates T cell proliferation [GO:0042098] Subtypes: negative regulation of immature T cell proliferation [GO:0033087], GO:0046007, negative regulation of T cell homeostatic proliferation [GO:0046014], negative regulation of alpha-beta T cell proliferation [GO:0046642], GO:0046647